hydroxymate-containing siderophore biosynthetic process [GO:0019539] (biological process) Definition: The chemical reactions and pathways resulting in the formation of a siderophore from other compounds, including hydroxamic acid. Hydroxamate is one of the three major chemical groups incorporated into siderophore structures with catechol and a-hydroxycarboxylate, each having a high selectivity for iron(3+). Subtypes: GO:0031169 Relationships: is a type of siderophore biosynthetic process [GO:0019290] References: PMID:20376388